{
  "gene_name": "Ubiquitin-like modifier-activating enzyme ATG7",
  "gene_symbol": "ATG7",
  "term_label": "autophagosome assembly",
  "gene": "UniProtKB:O95352",
  "term_id": "GO:0000045"
}